{
  "gene": "UniProtKB:Q96SZ6",
  "gene_symbol": "CDK5RAP1",
  "term_label": "mitochondrial tRNA modification",
  "gene_name": "Mitochondrial tRNA methylthiotransferase CDK5RAP1",
  "term_id": "GO:0070900"
}